protein import into peroxisome matrix, receptor recycling [GO:0016562] (BP) Definition: The process in which peroxisome targeting sequence receptors dissociates from cargo proteins and are returned to the cytosol. References: PMID:11687502 Also known as: peroxisome matrix protein import, receptor recycling, protein transport into peroxisome matrix, receptor recycling, receptor recycling during peroxisome matrix protein import, receptor recycling during protein import into peroxisome matrix, receptor recycling during protein transport into peroxisome matrix, PTS receptor recycling, peroxisome receptor recycling Relationships: is a type of GO:0001881; is part of GO:0016558